{
  "term_label": "myelin sheath",
  "term_id": "GO:0043209",
  "gene": "UniProtKB:P0DP23",
  "gene_name": "Calmodulin-1",
  "gene_symbol": "CALM1"
}